amygdalin beta-glucosidase activity [GO:0047668] (molecular function) Definition: Catalysis of the reaction: (R)-amygdalin + H2O = (R)-prunasin + D-glucose. Sources: EC:3.2.1.117, RHEA:14177 Relationships: is a type of GO:0008422 Also known as: amygdalinase, (R)-amygdalin beta-glucosidase activity, amygdalin b-glucosidase activity, amygdalin beta-D-glucohydrolase activity, amygdalin glucosidase activity, amygdalin hydrolase activity